{
  "term_label": "Unknown biological process",
  "gene_name": "Uncharacterized protein CXorf38",
  "gene_symbol": "CXorf38",
  "gene": "UniProtKB:Q8TB03",
  "term_id": "UNKNOWN:0002"
}